negative regulation of actin filament severing [GO:1903919] (biological process) References: PMID:23325791 Sources: GOC:TermGenie, GOC:als, GO_REF:0000058 Also known as: down regulation of F-actin severing, down regulation of actin filament severing, down-regulation of F-actin severing, down-regulation of actin filament severing, downregulation of F-actin severing, downregulation of actin filament severing, negative regulation of F-actin severing, inhibition of F-actin severing, inhibition of actin filament severing, down regulation of actin filament severing activity, down regulation of barbed-end actin capping/severing activity, down-regulation of actin filament severing activity, down-regulation of barbed-end actin capping/severing activity, downregulation of actin filament severing activity, downregulation of barbed-end actin capping/severing activity, inhibition of actin filament severing activity, inhibition of barbed-end actin capping/severing activity, negative regulation of actin filament severing activity, negative regulation of barbed-end actin capping/severing activity Relationships: is a type of negative regulation of cellular process [GO:0048523]; is a type of regulation of actin filament severing [GO:1903918]; negatively regulates actin filament severing [GO:0051014] Definition: Any process that stops, prevents or reduces the frequency, rate or extent of actin filament severing.